{
  "gene_symbol": "SYCE1L",
  "term_label": "Unknown biological process",
  "term_id": "UNKNOWN:0002",
  "gene_name": "Synaptonemal complex central element protein 1-like",
  "gene": "UniProtKB:A8MT33"
}